{
  "gene": "UniProtKB:A0A1W2PRE2",
  "gene_symbol": "A0A1W2PRE2",
  "gene_name": "Uncharacterized protein",
  "term_id": "UNKNOWN:0001",
  "term_label": "Unknown molecular function"
}